{
  "gene_name": "Zinc-alpha-2-glycoprotein",
  "term_id": "GO:0009897",
  "gene_symbol": "AZGP1",
  "term_label": "external side of plasma membrane",
  "gene": "UniProtKB:P25311"
}